positive regulation of calcium ion transmembrane transport [GO:1904427] (biological process) Definition: Any process that activates or increases the frequency, rate or extent of calcium ion transmembrane transport. References: PMID:22910094 Sources: GOC:TermGenie, GO_REF:0000058 Also known as: positive regulation of calcium ion membrane transport, positive regulation of transmembrane calcium transport, up regulation of calcium ion membrane transport, up regulation of calcium ion transmembrane transport, up regulation of transmembrane calcium transport, up-regulation of calcium ion membrane transport, up-regulation of calcium ion transmembrane transport, up-regulation of transmembrane calcium transport, upregulation of calcium ion membrane transport, upregulation of calcium ion transmembrane transport, upregulation of transmembrane calcium transport, activation of calcium ion membrane transport, activation of calcium ion transmembrane transport, activation of transmembrane calcium transport Relationships: is_a positive regulation of calcium ion transport [GO:0051928]; is a type of regulation of calcium ion transmembrane transport [GO:1903169]; is_a positive regulation of cation transmembrane transport [GO:1904064]; positively regulates calcium ion transmembrane transport [GO:0070588] Subtypes: positive regulation of calcium ion transport into cytosol [GO:0010524], positive regulation of release of sequestered calcium ion into cytosol [GO:0051281], positive regulation of calcium import into the mitochondrion [GO:0110098], positive regulation of calcium ion transmembrane transport via high voltage-gated calcium channel [GO:1904879], GO:1905665, positive regulation of calcium ion export across plasma membrane [GO:1905914]